{
  "term_label": "cytosol",
  "gene": "UniProtKB:Q96HD9",
  "gene_name": "N-acyl-aromatic-L-amino acid amidohydrolase (carboxylate-forming)",
  "gene_symbol": "ACY3",
  "term_id": "GO:0005829"
}